{
  "gene_symbol": "FRMD6-AS1",
  "gene": "UniProtKB:P0C7T7",
  "gene_name": "Putative uncharacterized protein FRMD6-AS1",
  "term_id": "UNKNOWN:0002",
  "term_label": "Unknown biological process"
}